{
  "gene_symbol": "ZDHHC9",
  "term_label": "Golgi apparatus",
  "term_id": "GO:0005794",
  "gene": "UniProtKB:Q9Y397",
  "gene_name": "Palmitoyltransferase ZDHHC9"
}